N-terminal peptidyl-glycine N-myristoylation [GO:0018008] (biological process) Definition: The myristoylation of the N-terminal glycine of proteins to form the derivative N-myristoyl-glycine. Sources: RESID:AA0059 Also known as: N-terminal peptidyl-glycine N-myristylation Relationships: is a type of N-terminal protein myristoylation [GO:0006499]; is a type of peptidyl-glycine modification [GO:0018201]